symbiont genome ejection through host cell envelope, long flexible tail mechanism [GO:0099001] (biological process) Relationships: is a type of GO:0039678 Also known as: viral long flexible tail ejection system, viral genome ejection through host cell envelope, long flexible tail mechanism References: PMID:22297512 Sources: GOC:dos, VZ:3952 Definition: Entry of a symbiont's genome into the host cell through the host cell envelope via a long, flexible tail ejection system consisting a baseplate, a central tube and a terminator complex which attaches the tail to the phage capsid. Upon binding to the host cell surface, the baseplate changes its conformation and triggers genome ejection into the host cell cytoplasm. Occurs in non-enveloped prokaryotic viruses.